{
  "gene_symbol": "DDX3Y",
  "term_id": "GO:0005634",
  "gene": "UniProtKB:O15523",
  "gene_name": "ATP-dependent RNA helicase DDX3Y",
  "term_label": "nucleus"
}